{
  "gene_symbol": "OXSM",
  "term_label": "mitochondrion",
  "gene_name": "3-oxoacyl-[acyl-carrier-protein] synthase, mitochondrial",
  "gene": "UniProtKB:Q9NWU1",
  "term_id": "GO:0005739"
}